{
  "term_id": "GO:0006612",
  "gene": "UniProtKB:Q9NYG2",
  "gene_symbol": "ZDHHC3",
  "term_label": "protein targeting to membrane",
  "gene_name": "Palmitoyltransferase ZDHHC3"
}